{
  "gene_symbol": "LSM1",
  "term_id": "GO:0000932",
  "gene": "UniProtKB:O15116",
  "term_label": "P-body",
  "gene_name": "U6 snRNA-associated Sm-like protein LSm1"
}